{
  "term_label": "purine nucleoside metabolic process",
  "gene": "UniProtKB:A1Z1Q3",
  "gene_symbol": "MACROD2",
  "term_id": "GO:0042278",
  "gene_name": "ADP-ribose glycohydrolase MACROD2"
}